{
  "gene_symbol": "C7orf50",
  "term_label": "Unknown cellular component",
  "term_id": "UNKNOWN:0003",
  "gene_name": "Uncharacterized protein C7orf50",
  "gene": "UniProtKB:Q9BRJ6"
}